transposase activity [GO:0004803] (molecular function) Also known as: P-element encoded transposase activity Relationships: is a type of GO:0140097 Definition: Catalysis of the transposition of transposable elements or transposons. Transposases are involved in recombination required for transposition and are site-specific for the transposon/transposable element. Sources: GOC:bm, ISBN:0198506732